secretin receptor binding [GO:0031876] (molecular function) Also known as: secretin receptor ligand Relationships: is_a G protein-coupled receptor binding [GO:0001664] Definition: Binding to a secretin receptor. Sources: GOC:mah, GOC:nln